pectin biosynthetic process [GO:0045489] (BP) Definition: The chemical reactions and pathways resulting in the formation of pectin, a polymer containing a backbone of alpha-1,4-linked D-galacturonic acid residues. Also known as: pectin anabolism, pectin biosynthesis, pectin formation, pectin synthesis Subtypes: GO:0048358, cell wall pectin biosynthetic process [GO:0052325] Relationships: is a type of GO:0000271; is a type of pectin metabolic process [GO:0045488] Regulation: regulated by regulation of pectin biosynthetic process [GO:1900030] References: PMID:11931668 Sources: GOC:go_curators